{
  "gene_symbol": "IFT22",
  "gene_name": "Intraflagellar transport protein 22 homolog",
  "term_label": "intracellular protein transport",
  "term_id": "GO:0006886",
  "gene": "UniProtKB:Q9H7X7"
}